chylomicron remodeling [GO:0034371] (biological process) Definition: The acquisition, loss or modification of a protein or lipid within a chylomicron, including the hydrolysis of triglyceride by lipoprotein lipase and the subsequent loss of free fatty acid. Also known as: chylomicron remodelling, chylomicron remnant formation Relationships: is a type of triglyceride-rich lipoprotein particle remodeling [GO:0034370] Sources: GOC:BHF, GOC:expert_pt, GOC:mah, GOC:rl Regulation: regulated by GO:0090318; positively regulated by positive regulation of chylomicron remodeling [GO:0090319]